{
  "gene_name": "Cytoplasmic dynein 2 intermediate chain 1",
  "gene": "UniProtKB:Q8WVS4",
  "gene_symbol": "DYNC2I1",
  "term_id": "GO:0060271",
  "term_label": "cilium assembly"
}